{
  "gene_name": "Beta-crystallin A4",
  "gene_symbol": "CRYBA4",
  "term_id": "GO:0005212",
  "gene": "UniProtKB:P53673",
  "term_label": "structural constituent of eye lens"
}